{
  "term_label": "lens development in camera-type eye",
  "gene_symbol": "CRYBB2",
  "term_id": "GO:0002088",
  "gene_name": "Beta-crystallin B2",
  "gene": "UniProtKB:P43320"
}